{
  "term_id": "UNKNOWN:0002",
  "term_label": "Unknown biological process",
  "gene_name": "Large ribosomal subunit protein mL45",
  "gene_symbol": "MRPL45",
  "gene": "UniProtKB:Q9BRJ2"
}